{
  "term_label": "acetylgalactosaminyltransferase activity",
  "gene_symbol": "B4GALNT3",
  "term_id": "GO:0008376",
  "gene": "UniProtKB:Q6L9W6",
  "gene_name": "Beta-1,4-N-acetylgalactosaminyltransferase 3"
}